{
  "gene_symbol": "UBE2G2",
  "term_label": "cytosol",
  "gene": "UniProtKB:P60604",
  "gene_name": "Ubiquitin-conjugating enzyme E2 G2",
  "term_id": "GO:0005829"
}